cyclic nucleotide-dependent protein kinase activity [GO:0004690] (molecular function) Sources: GOC:mah Subtypes: cAMP-dependent protein kinase activity [GO:0004691], GO:0004692 Definition: cNMP-dependent catalysis of the reaction: ATP + a protein = ADP + a phosphoprotein. Note: This reaction requires the presence of a cyclic nucleotide. Relationships: is a type of protein serine/threonine kinase activity [GO:0004674]; has part cyclic nucleotide binding [GO:0030551]